{
  "term_id": "UNKNOWN:0002",
  "term_label": "Unknown biological process",
  "gene_name": "Immortalization up-regulated protein",
  "gene": "UniProtKB:Q9GZP8",
  "gene_symbol": "IMUP"
}